anterior/posterior pattern specification involved in ureteric bud development [GO:0072099] (BP) Also known as: ureteric bud anterior/posterior pattern formation Subtypes: specification of ureteric bud anterior/posterior symmetry [GO:0072100] Relationships: is a type of pattern specification involved in mesonephros development [GO:0061227]; is a type of GO:0072098; is part of ureteric bud development [GO:0001657] Definition: The developmental process that results in the creation of defined areas or spaces within the ureteric bud along the anterior/posterior axis to which cells respond and eventually are instructed to differentiate. Sources: GOC:mtg_kidney_jan10